posterior compartment specification [GO:0007388] (BP) Definition: The process involved in the specification of cell identity in the posterior compartments of the segmented embryo. Relationships: is a type of GO:0007386 Sources: ISBN:0879694238, http://fly.ebi.ac.uk/allied-data/lk/interactive-fly/aimain/1aahome.htm